{
  "gene_symbol": "PRKCD",
  "term_id": "GO:0035556",
  "gene_name": "Protein kinase C delta type",
  "term_label": "intracellular signal transduction",
  "gene": "UniProtKB:Q05655"
}